{
  "term_id": "GO:0061630",
  "gene": "UniProtKB:Q8WVZ7",
  "gene_symbol": "RNF133",
  "term_label": "ubiquitin protein ligase activity",
  "gene_name": "E3 ubiquitin-protein ligase RNF133"
}